SCF-dependent proteasomal ubiquitin-dependent protein catabolic process [GO:0031146] (biological process) References: PMID:15380083 Regulation: regulated by GO:0062025; RO_0002212 by negative regulation of SCF-dependent proteasomal ubiquitin-dependent catabolic process [GO:0062026]; positively regulated by positive regulation of SCF-dependent proteasomal ubiquitin-dependent catabolic process [GO:0062027] Also known as: SCF-dependent proteasomal ubiquitin-dependent protein breakdown, SCF-dependent proteasomal ubiquitin-dependent protein catabolism, SCF-dependent proteasomal ubiquitin-dependent protein degradation Definition: The chemical reactions and pathways resulting in the breakdown of a protein or peptide by hydrolysis of its peptide bonds, initiated by the covalent attachment of ubiquitin, with ubiquitin-protein ligation catalyzed by an SCF (Skp1/Cul1/F-box protein) complex, and mediated by the proteasome. Relationships: is a type of GO:0043161